{
  "gene": "UniProtKB:Q9UDY2",
  "gene_name": "Tight junction protein ZO-2",
  "term_id": "GO:0005923",
  "gene_symbol": "TJP2",
  "term_label": "bicellular tight junction"
}